{
  "gene_name": "Zinc finger protein 655",
  "gene": "UniProtKB:Q8N720",
  "term_label": "RNA polymerase II cis-regulatory region sequence-specific DNA binding",
  "term_id": "GO:0000978",
  "gene_symbol": "ZNF655"
}